{
  "term_label": "extracellular space",
  "term_id": "GO:0005615",
  "gene_name": "Semenogelin-2",
  "gene": "UniProtKB:Q02383",
  "gene_symbol": "SEMG2"
}